{
  "gene": "UniProtKB:Q13033",
  "gene_symbol": "STRN3",
  "term_id": "GO:0043025",
  "gene_name": "Striatin-3",
  "term_label": "neuronal cell body"
}